{
  "gene_name": "Helicase POLQ-like",
  "term_label": "DNA double-strand break processing involved in repair via single-strand annealing",
  "term_id": "GO:0010792",
  "gene": "UniProtKB:Q8TDG4",
  "gene_symbol": "HELQ"
}